{
  "gene_symbol": "PSPN",
  "term_label": "glial cell-derived neurotrophic factor receptor signaling pathway",
  "gene_name": "Persephin",
  "term_id": "GO:0035860",
  "gene": "UniProtKB:O60542"
}